{
  "gene_name": "Mucin-17",
  "term_id": "UNKNOWN:0001",
  "gene_symbol": "MUC17",
  "term_label": "Unknown molecular function",
  "gene": "UniProtKB:Q685J3"
}